{
  "gene": "UniProtKB:Q8WYJ6",
  "term_label": "cytoskeleton-dependent cytokinesis",
  "gene_name": "Septin-1",
  "term_id": "GO:0061640",
  "gene_symbol": "SEPTIN1"
}